{
  "term_label": "SCF-dependent proteasomal ubiquitin-dependent protein catabolic process",
  "gene_name": "S-phase kinase-associated protein 1",
  "gene_symbol": "SKP1",
  "term_id": "GO:0031146",
  "gene": "UniProtKB:P63208"
}